{
  "gene": "UniProtKB:Q96N38",
  "gene_name": "Zinc finger protein 714",
  "gene_symbol": "ZNF714",
  "term_label": "regulation of DNA-templated transcription",
  "term_id": "GO:0006355"
}